{
  "gene_name": "Mediator of RNA polymerase II transcription subunit 1",
  "term_id": "GO:0006357",
  "term_label": "regulation of transcription by RNA polymerase II",
  "gene_symbol": "MED1",
  "gene": "UniProtKB:Q15648"
}